{
  "gene_name": "Mitochondrial brown fat uncoupling protein 1",
  "gene": "UniProtKB:P25874",
  "term_label": "mitochondrial inner membrane",
  "term_id": "GO:0005743",
  "gene_symbol": "UCP1"
}